{
  "term_label": "regulation of sodium ion transport",
  "gene_name": "Sodium_potassium-transporting ATPase subunit beta-1-interacting protein 3",
  "gene_symbol": "NKAIN3",
  "term_id": "GO:0002028",
  "gene": "UniProtKB:Q8N8D7"
}